{
  "term_label": "fatty acid synthase activity",
  "gene": "UniProtKB:P49327",
  "term_id": "GO:0004312",
  "gene_name": "Fatty acid synthase",
  "gene_symbol": "FASN"
}